{
  "gene_symbol": "CLEC4E",
  "term_label": "antifungal innate immune response",
  "gene_name": "C-type lectin domain family 4 member E",
  "gene": "UniProtKB:Q9ULY5",
  "term_id": "GO:0061760"
}